{
  "gene": "UniProtKB:P00748",
  "term_label": "rough endoplasmic reticulum",
  "term_id": "GO:0005791",
  "gene_symbol": "F12",
  "gene_name": "Coagulation factor XII"
}